{
  "gene": "UniProtKB:Q8N816",
  "term_id": "UNKNOWN:0002",
  "gene_symbol": "KRT10-AS1",
  "term_label": "Unknown biological process",
  "gene_name": "Uncharacterized protein KRT10-AS1"
}